{
  "gene_name": "Rho guanine nucleotide exchange factor 28",
  "term_id": "GO:0035023",
  "gene_symbol": "ARHGEF28",
  "term_label": "regulation of Rho protein signal transduction",
  "gene": "UniProtKB:Q8N1W1"
}